{
  "gene_name": "Keratin, type I cuticular Ha3-II",
  "gene_symbol": "KRT33B",
  "term_id": "GO:0030855",
  "gene": "UniProtKB:Q14525",
  "term_label": "epithelial cell differentiation"
}